regulation of tolerance induction dependent upon immune response [GO:0002652] (biological process) Also known as: regulation of immune response-dependent tolerance induction Definition: Any process that modulates the frequency, rate, or extent of tolerance induction dependent upon immune response. Subtypes: negative regulation of tolerance induction dependent upon immune response [GO:0002653], positive regulation of tolerance induction dependent upon immune response [GO:0002654], regulation of tolerance induction to nonself antigen [GO:0002655], GO:0002658 Relationships: is a type of regulation of tolerance induction [GO:0002643]; is a type of regulation of adaptive immune response based on somatic recombination of immune receptors built from immunoglobulin superfamily domains [GO:0002822]; RO_0002211 GO:0002461 Sources: GOC:add